{
  "gene_name": "Phosphatidate phosphatase LPIN1",
  "term_id": "GO:0003713",
  "gene_symbol": "LPIN1",
  "gene": "UniProtKB:Q14693",
  "term_label": "transcription coactivator activity"
}